Sid2-Mob1 complex [GO:0034973] (cellular component) Relationships: is a type of GO:0032991; is part of cytoplasm [GO:0005737] Also known as: Dbf2p-Mob1p complex, Sid2-Mob1 kinase complex, Sid2p-Mob1p complex References: PMID:10837231, PMID:15060149 Sources: GOC:vw Definition: A protein complex that contains a protein kinase (Sid2 in S. pombe) and its regulatory subunit (Mob1). The Sid2p-Mob1p kinase complex is a component of the septation initiation network in fission yeast (called the mitotic exit network in S. cerevisiae) and is required for cytokinesis. The analogous complex in S. cerevisiae is called Dbf2p-Mob1p complex.